{
  "gene_symbol": "CREB3L4",
  "gene": "UniProtKB:Q8TEY5",
  "term_id": "GO:0000978",
  "gene_name": "Cyclic AMP-responsive element-binding protein 3-like protein 4",
  "term_label": "RNA polymerase II cis-regulatory region sequence-specific DNA binding"
}